{
  "gene_name": "Putative olfactory receptor 2B3",
  "term_id": "GO:0004984",
  "term_label": "olfactory receptor activity",
  "gene_symbol": "OR2B3",
  "gene": "UniProtKB:O76000"
}